glossopharyngeal nerve morphogenesis [GO:0021615] (biological process) Definition: The process in which the anatomical structure of the glossopharyngeal nerve is generated and organized. Various sensory and motor branches of the glossopharyngeal nerve supply nerve connections to the pharynx and back of the tongue. The branchial motor component contains motor fibers that innervate muscles that elevate the pharynx and larynx, and the tympanic branch supplies parasympathetic fibers to the otic ganglion. Relationships: is a type of cranial nerve morphogenesis [GO:0021602]; is part of GO:0021563 Also known as: CN IX morphogenesis Sources: GOC:cls, GOC:dgh, GOC:dph, GOC:jid, GO_REF:0000021